negative regulation of phosphatidic acid biosynthetic process [GO:1905694] (biological process) References: PMID:23767959 Sources: GOC:PARL, GOC:TermGenie, GOC:bc, GO_REF:0000058 Definition: Any process that stops, prevents or reduces the frequency, rate or extent of phosphatidic acid biosynthetic process. Also known as: down regulation of phosphatidic acid anabolism, down regulation of phosphatidic acid biosynthesis, down regulation of phosphatidic acid biosynthetic process, down regulation of phosphatidic acid formation, down regulation of phosphatidic acid synthesis, down-regulation of phosphatidic acid anabolism, down-regulation of phosphatidic acid biosynthesis, down-regulation of phosphatidic acid biosynthetic process, down-regulation of phosphatidic acid formation, down-regulation of phosphatidic acid synthesis, downregulation of phosphatidic acid anabolism, downregulation of phosphatidic acid biosynthesis, downregulation of phosphatidic acid biosynthetic process, downregulation of phosphatidic acid formation, downregulation of phosphatidic acid synthesis, negative regulation of phosphatidic acid anabolism, negative regulation of phosphatidic acid biosynthesis, negative regulation of phosphatidic acid formation, negative regulation of phosphatidic acid synthesis, inhibition of phosphatidic acid anabolism, inhibition of phosphatidic acid biosynthesis, inhibition of phosphatidic acid biosynthetic process, inhibition of phosphatidic acid formation, inhibition of phosphatidic acid synthesis Relationships: is a type of negative regulation of phospholipid biosynthetic process [GO:0071072]; is a type of GO:1905693; negatively regulates GO:0006654